{
  "gene_name": "Kinesin-like protein KIF9",
  "gene_symbol": "KIF9",
  "term_id": "GO:0016887",
  "term_label": "ATP hydrolysis activity",
  "gene": "UniProtKB:Q9HAQ2"
}